{
  "gene": "UniProtKB:Q14162",
  "gene_name": "Scavenger receptor class F member 1",
  "term_id": "GO:0016358",
  "gene_symbol": "SCARF1",
  "term_label": "dendrite development"
}